{
  "term_id": "GO:0005737",
  "gene_name": "Prostamide_prostaglandin F synthase",
  "gene": "UniProtKB:Q8TBF2",
  "term_label": "cytoplasm",
  "gene_symbol": "PRXL2B"
}